{
  "term_label": "regulation of calcineurin-NFAT signaling cascade",
  "gene_name": "EF-hand domain-containing family member B",
  "gene_symbol": "EFHB",
  "term_id": "GO:0070884",
  "gene": "UniProtKB:Q8N7U6"
}